{
  "term_label": "cell differentiation",
  "gene_name": "Friend leukemia integration 1 transcription factor",
  "gene": "UniProtKB:Q01543",
  "gene_symbol": "FLI1",
  "term_id": "GO:0030154"
}